{
  "gene_name": "Interferon-related developmental regulator 2",
  "gene": "UniProtKB:Q12894",
  "gene_symbol": "IFRD2",
  "term_label": "Unknown molecular function",
  "term_id": "UNKNOWN:0001"
}